{
  "gene_symbol": "FOSB",
  "gene_name": "Protein FosB",
  "gene": "UniProtKB:P53539",
  "term_id": "GO:0006357",
  "term_label": "regulation of transcription by RNA polymerase II"
}